{
  "term_id": "GO:0005634",
  "gene_symbol": "PLK3",
  "term_label": "nucleus",
  "gene": "UniProtKB:Q9H4B4",
  "gene_name": "Serine_threonine-protein kinase PLK3"
}